{
  "gene_symbol": "PARD3B",
  "term_label": "apical plasma membrane",
  "gene_name": "Partitioning defective 3 homolog B",
  "gene": "UniProtKB:Q8TEW8",
  "term_id": "GO:0016324"
}